RISC complex assembly [GO:0070922] (biological process) Definition: The process in which a single-stranded small RNA is incorporated within the RNA-initiated silencing complex (RISC). The assembly includes the maturation of the small RNA, the stabilization of the complex by accessory proteins of the RISC complex, duplex separation and the release of the second strand, forming a base-pairing complement complex that mediates gene silencing by small RNA. References: PMID:14512631, PMID:14744438, PMID:19239886, PMID:22233755, PMID:27184117 Also known as: miRISC assembly, miRNA loading onto RISC, siRNA loading onto RISC involved in RNA interference, siRNA loading onto RISC involved in gene silencing by small RNA, RISC assembly, gene silencing by RNA, small RNA loading onto RISC, small RNA loading onto RISC Relationships: is a type of protein-RNA complex assembly [GO:0022618]; BFO_0000050 GO:0031047